{
  "gene_name": "Globoside alpha-1,3-N-acetylgalactosaminyltransferase 1",
  "gene": "UniProtKB:Q8N5D6",
  "term_id": "UNKNOWN:0002",
  "gene_symbol": "GBGT1",
  "term_label": "Unknown biological process"
}